{
  "term_id": "UNKNOWN:0003",
  "gene_name": "SHC SH2 domain-binding protein 1",
  "term_label": "Unknown cellular component",
  "gene_symbol": "SHCBP1",
  "gene": "UniProtKB:Q8NEM2"
}